{
  "gene_name": "Cyclin-A2",
  "term_label": "cyclin-dependent protein serine/threonine kinase regulator activity",
  "gene": "UniProtKB:P20248",
  "term_id": "GO:0016538",
  "gene_symbol": "CCNA2"
}